{
  "gene": "UniProtKB:Q9C0D3",
  "term_id": "UNKNOWN:0002",
  "gene_name": "Protein zyg-11 homolog B",
  "term_label": "Unknown biological process",
  "gene_symbol": "ZYG11B"
}